{
  "gene_symbol": "NKD2",
  "term_label": "cytoplasm",
  "term_id": "GO:0005737",
  "gene": "UniProtKB:Q969F2",
  "gene_name": "Protein naked cuticle homolog 2"
}